{
  "term_label": "SNAP receptor activity",
  "term_id": "GO:0005484",
  "gene_name": "Golgi SNAP receptor complex member 1",
  "gene_symbol": "GOSR1",
  "gene": "UniProtKB:O95249"
}